{
  "gene_name": "Muscarinic acetylcholine receptor M3",
  "gene_symbol": "CHRM3",
  "gene": "UniProtKB:P20309",
  "term_id": "GO:0005886",
  "term_label": "plasma membrane"
}